positive regulation of cyanophore differentiation [GO:0048783] (biological process) Definition: Any process that activates or increases the frequency, rate or extent of cyanophore differentiation. Sources: GOC:mh Also known as: up regulation of cyanophore differentiation, up-regulation of cyanophore differentiation, upregulation of cyanophore differentiation, activation of cyanophore differentiation, stimulation of cyanophore differentiation Relationships: is a type of regulation of cyanophore differentiation [GO:0048781]; is a type of GO:0050942; positively regulates GO:0048774